{
  "gene_name": "Centrosomal protein of 120 kDa",
  "term_label": "Unknown molecular function",
  "term_id": "UNKNOWN:0001",
  "gene": "UniProtKB:Q8N960",
  "gene_symbol": "CEP120"
}